{
  "gene_symbol": "SLFN5",
  "gene": "UniProtKB:Q08AF3",
  "term_id": "UNKNOWN:0003",
  "term_label": "Unknown cellular component",
  "gene_name": "Schlafen family member 5"
}